negative regulation of cell communication [GO:0010648] (biological process) Relationships: is_a regulation of cell communication [GO:0010646]; is a type of negative regulation of cellular process [GO:0048523]; negatively regulates GO:0007154 Definition: Any process that decreases the frequency, rate or extent of cell communication. Cell communication is the process that mediates interactions between a cell and its surroundings. Encompasses interactions such as signaling or attachment between one cell and another cell, between a cell and an extracellular matrix, or between a cell and any other aspect of its environment. Subtypes: negative regulation of signal transduction [GO:0009968], GO:0010651, negative regulation of cell communication by chemical coupling [GO:0010653], GO:0046888, GO:0050805, negative regulation of transmission of nerve impulse [GO:0051970], negative regulation of Wnt protein secretion [GO:0061358], negative regulation of c-di-GMP signaling [GO:0061942], negative regulation of trichome patterning [GO:1900033], negative regulation of retrograde trans-synaptic signaling by neuropeptide [GO:1905433], negative regulation of BMP secretion [GO:2001285] Sources: GOC:dph, GOC:tb